{
  "gene": "UniProtKB:Q9UNK0",
  "gene_name": "Syntaxin-8",
  "term_id": "GO:0012505",
  "term_label": "endomembrane system",
  "gene_symbol": "STX8"
}